regulation of primary miRNA processing [GO:2000634] (biological process) Relationships: is a type of regulation of miRNA processing [GO:1903798]; regulates primary miRNA processing [GO:0031053] Sources: GOC:dph, GOC:sl Definition: Any process that modulates the frequency, rate or extent of primary microRNA processing. Subtypes: GO:2000635, positive regulation of primary miRNA processing [GO:2000636] Also known as: regulation of pri-miRNA processing, regulation of primary microRNA processing